dolichyl monophosphate biosynthetic process [GO:0043048] (biological process) Regulation: regulated by GO:0010794 References: PMID:21384228, PMID:38821050 Sources: MetaCyc:PWY-6129 Definition: The chemical reactions and pathways resulting in the formation of dolichyl monophosphate, a phosphorylated dolichol derivative. Also known as: dolichyl monophosphate anabolism, dolichyl monophosphate biosynthesis, dolichyl monophosphate formation, dolichyl monophosphate synthesis Relationships: is a type of phospholipid biosynthetic process [GO:0008654]